exit of virus from host cell nucleus by nuclear egress [GO:0046802] (BP) Also known as: capsid egress, nuclear egress, nuclear egress of viral procapsid, egress of viral procapsid from host cell nucleus Relationships: is a type of exit of virus from host cell nucleus [GO:0039674] References: PMID:21494278, PMID:22858153, PMID:9601512, PMID:9765421 Sources: VZ:1952 Definition: The directed movement of an assembled viral particle out of the host cell nucleus by budding and fusion through the nuclear membranes. In this process, enveloped viral particles are formed by budding through the inner nuclear membrane. These perinuclear enveloped particles then fuse with the outer nuclear membrane to deliver a naked capsid into the host cytoplasm.